{
  "term_id": "GO:0004984",
  "gene": "UniProtKB:Q8NH42",
  "term_label": "olfactory receptor activity",
  "gene_name": "Olfactory receptor 4K13",
  "gene_symbol": "OR4K13"
}